voltage-gated sodium channel activity involved in SA node cell action potential [GO:0086063] (MF) Also known as: voltage-gated sodium channel activity involved in SA node cardiac muscle cell action potential, voltage-gated sodium channel activity involved in SAN cardiac muscle cell action potential, voltage-gated sodium channel activity involved in sinoatrial node cardiac muscle cell action potential, voltage-gated sodium channel activity involved in sinus node cardiac muscle cell action potential Definition: Enables the transmembrane transfer of a sodium ion by a voltage-gated channel through the plasma membrane of an SA node cardiac muscle cell contributing to the depolarization phase of an action potential. A voltage-gated channel is a channel whose open state is dependent on the voltage across the membrane in which it is embedded. Relationships: is a type of voltage-gated sodium channel activity involved in cardiac muscle cell action potential [GO:0086006]; is part of membrane depolarization during SA node cell action potential [GO:0086046] Sources: GOC:BHF, GOC:mtg_cardiac_conduct_nov11